{
  "term_label": "protein-macromolecule adaptor activity",
  "gene": "UniProtKB:Q9HAP6",
  "gene_name": "Protein lin-7 homolog B",
  "gene_symbol": "LIN7B",
  "term_id": "GO:0030674"
}